{
  "gene_name": "Extracellular sulfatase Sulf-2",
  "term_id": "GO:0005615",
  "gene_symbol": "SULF2",
  "gene": "UniProtKB:Q8IWU5",
  "term_label": "extracellular space"
}